cyanophore differentiation [GO:0048774] (biological process) Definition: The process in which a relatively unspecialized cell acquires the specialized features of a cyanophore cell. Cyanophores are pigment cells derived from the neural crest. They contain a blue pigment of unknown chemical composition. The pigment is stored in fibrous organelles termed cyanosomes. Sources: GOC:jid, GOC:mh Also known as: cyanophore cell differentiation Relationships: is a type of pigment cell differentiation [GO:0050931] Regulation: regulated by regulation of cyanophore differentiation [GO:0048781]; negatively regulated by negative regulation of cyanophore differentiation [GO:0048782]; RO_0002213 by positive regulation of cyanophore differentiation [GO:0048783]